positive regulation of embryonic development [GO:0040019] (biological process) Definition: Any process that activates or increases the frequency, rate or extent of embryonic development. Sources: GOC:go_curators Relationships: is a type of regulation of embryonic development [GO:0045995]; is a type of positive regulation of developmental process [GO:0051094]; is a type of GO:0051240; positively regulates embryo development [GO:0009790] Subtypes: GO:0061184, positive regulation of gastrulation [GO:2000543] Also known as: up regulation of embryonic development, up-regulation of embryonic development, upregulation of embryonic development, activation of embryonic development, stimulation of embryonic development